facial nerve maturation [GO:0021613] (biological process) Definition: A developmental process, independent of morphogenetic (shape) change, that is required for the facial nerve to attain its fully functional state. This sensory and motor nerve supplies the muscles of facial expression and the expression and taste at the anterior two-thirds of the tongue. The principal branches are the superficial ophthalmic, buccal, palatine and hyomandibular. The main trunk synapses within pterygopalatine ganglion in the parotid gland and this ganglion then gives of nerve branches which supply the lacrimal gland and the mucous secreting glands of the nasal and oral cavities. Sources: GOC:cls, GOC:dgh, GOC:dph, GOC:jid, GO_REF:0000021 Also known as: CN VII maturation Relationships: is a type of cranial nerve maturation [GO:0021605]; is part of facial nerve development [GO:0021561]